{
  "term_id": "UNKNOWN:0003",
  "gene": "UniProtKB:A0A1B0GVG6",
  "gene_symbol": "TEX54",
  "gene_name": "Testis-expressed protein 54",
  "term_label": "Unknown cellular component"
}